{
  "term_label": "membrane",
  "gene_symbol": "KCNU1",
  "gene": "UniProtKB:A8MYU2",
  "gene_name": "Potassium channel subfamily U member 1",
  "term_id": "GO:0016020"
}